{
  "gene": "UniProtKB:Q9UNY5",
  "term_id": "UNKNOWN:0003",
  "gene_name": "Zinc finger protein 232",
  "term_label": "Unknown cellular component",
  "gene_symbol": "ZNF232"
}